D-glucuronate catabolic process [GO:0042840] (biological process) Relationships: is a type of glucuronate catabolic process [GO:0006064] Subtypes: D-glucuronate catabolic process to D-xylulose 5-phosphate [GO:0019640] Also known as: D-glucuronate breakdown, D-glucuronate catabolism, D-glucuronate degradation Definition: The chemical reactions and pathways resulting in the breakdown of D-glucuronate, the D-enantiomer of glucuronate. Sources: GOC:jl, GOC:jsg, GOC:mah